{
  "gene_symbol": "DCDC2B",
  "term_id": "GO:0005815",
  "term_label": "microtubule organizing center",
  "gene_name": "Doublecortin domain-containing protein 2B",
  "gene": "UniProtKB:A2VCK2"
}